{
  "gene_name": "Kelch-like protein 41",
  "term_label": "M band",
  "gene_symbol": "KLHL41",
  "term_id": "GO:0031430",
  "gene": "UniProtKB:O60662"
}